{
  "gene_symbol": "ZNF705A",
  "term_id": "GO:0000977",
  "gene_name": "Zinc finger protein 705A",
  "term_label": "RNA polymerase II transcription regulatory region sequence-specific DNA binding",
  "gene": "UniProtKB:Q6ZN79"
}